{
  "gene_name": "Probable ATP-dependent RNA helicase DDX46",
  "term_id": "UNKNOWN:0001",
  "gene": "UniProtKB:Q7L014",
  "gene_symbol": "DDX46",
  "term_label": "Unknown molecular function"
}